{
  "gene": "UniProtKB:P22352",
  "term_id": "GO:0008430",
  "gene_name": "Glutathione peroxidase 3",
  "term_label": "selenium binding",
  "gene_symbol": "GPX3"
}